{
  "term_id": "GO:0005739",
  "gene_symbol": "MRPL37",
  "term_label": "mitochondrion",
  "gene_name": "Large ribosomal subunit protein mL37",
  "gene": "UniProtKB:Q9BZE1"
}